{
  "gene_name": "Taperin",
  "gene_symbol": "TPRN",
  "term_label": "sensory perception of sound",
  "gene": "UniProtKB:Q4KMQ1",
  "term_id": "GO:0007605"
}